{
  "gene_symbol": "VPS36",
  "term_label": "late endosome membrane",
  "gene": "UniProtKB:Q86VN1",
  "gene_name": "Vacuolar protein-sorting-associated protein 36",
  "term_id": "GO:0031902"
}